{
  "gene": "UniProtKB:A1L020",
  "gene_symbol": "MEX3A",
  "term_label": "Unknown molecular function",
  "gene_name": "RNA-binding protein MEX3A",
  "term_id": "UNKNOWN:0001"
}